{
  "term_label": "negative regulation of synaptic vesicle exocytosis",
  "term_id": "GO:2000301",
  "gene": "UniProtKB:A6NIZ1",
  "gene_symbol": "RAP1BL",
  "gene_name": "Ras-related protein Rap-1b-like protein"
}